{
  "term_id": "GO:0110155",
  "gene_symbol": "DXO",
  "gene_name": "Decapping and exoribonuclease protein",
  "term_label": "NAD-cap decapping",
  "gene": "UniProtKB:O77932"
}